macromolecule modification [GO:0043412] (biological process) Definition: The covalent alteration of one or more monomeric units in a polypeptide, polynucleotide, polysaccharide, or other biological macromolecule, resulting in a change in its properties. Relationships: is a type of macromolecule metabolic process [GO:0043170] Sources: GOC:go_curators Subtypes: GO:0006304, GO:0009451, protein modification process [GO:0036211], macromolecule methylation [GO:0043414], sialylation [GO:0097503], macromolecule deacylation [GO:0098732]